{
  "gene": "UniProtKB:Q5SVZ6",
  "term_id": "UNKNOWN:0001",
  "gene_symbol": "ZMYM1",
  "term_label": "Unknown molecular function",
  "gene_name": "Zinc finger MYM-type protein 1"
}